anterograde dendritic transport of mitochondrion [GO:0098972] (biological process) Sources: GOC:dos Definition: The directed movement of mitochondria along microtubules in dendrites towards the postsynapse and away from the cell body. Relationships: is a type of anterograde dendritic transport [GO:0098937]; is a type of GO:0098939